{
  "gene_symbol": "AREL1",
  "gene_name": "Apoptosis-resistant E3 ubiquitin protein ligase 1",
  "term_label": "negative regulation of apoptotic process",
  "gene": "UniProtKB:O15033",
  "term_id": "GO:0043066"
}